{
  "gene_symbol": "PEBP4",
  "gene": "UniProtKB:Q96S96",
  "gene_name": "Phosphatidylethanolamine-binding protein 4",
  "term_label": "Unknown biological process",
  "term_id": "UNKNOWN:0002"
}